{
  "gene_symbol": "SLC12A2",
  "gene": "UniProtKB:P55011",
  "gene_name": "Solute carrier family 12 member 2",
  "term_id": "GO:0072488",
  "term_label": "ammonium transmembrane transport"
}